negative regulation of glucosylceramide biosynthetic process [GO:0046318] (biological process) Also known as: down regulation of glucosylceramide biosynthetic process, down-regulation of glucosylceramide biosynthetic process, downregulation of glucosylceramide biosynthetic process, negative regulation of glucosylceramide anabolism, negative regulation of glucosylceramide biosynthesis, negative regulation of glucosylceramide formation, negative regulation of glucosylceramide synthesis, inhibition of glucosylceramide biosynthetic process Sources: GOC:ai, GOC:ascb_2009, GOC:dph, GOC:tb Definition: Any process that stops, prevents, or reduces the frequency, rate or extent of the chemical reactions and pathways resulting in the formation of glucosylceramide. Relationships: is a type of regulation of glucosylceramide biosynthetic process [GO:0046317]; is_a negative regulation of ceramide biosynthetic process [GO:1900060]; negatively regulates glucosylceramide biosynthetic process [GO:0006679]